{
  "gene": "UniProtKB:Q9BPZ7",
  "term_label": "plasma membrane",
  "term_id": "GO:0005886",
  "gene_name": "Target of rapamycin complex 2 subunit MAPKAP1",
  "gene_symbol": "MAPKAP1"
}